acetyl-CoA metabolic process [GO:0006084] (biological process) Also known as: acetyl coenzyme A metabolic process, acetyl coenzyme A metabolism, acetyl-CoA metabolism Sources: ISBN:0198547684 Definition: The chemical reactions and pathways involving acetyl-CoA, a derivative of coenzyme A in which the sulfhydryl group is acetylated; it is a metabolite derived from several pathways (e.g. glycolysis, fatty acid oxidation, amino-acid catabolism) and is further metabolized by the tricarboxylic acid cycle. It is a key intermediate in lipid and terpenoid biosynthesis. Subtypes: acetyl-CoA biosynthetic process [GO:0006085], isopentenyl diphosphate biosynthetic process, mevalonate pathway [GO:0019287], L-tryptophan catabolic process to acetyl-CoA [GO:0019442], GO:0019474, butyryl-CoA biosynthetic process from acetyl-CoA [GO:0044579], acetyl-CoA catabolic process [GO:0046356], L-threonine catabolic process to acetyl-CoA [GO:0070690] Relationships: is a type of GO:0006637